{
  "gene_symbol": "ANXA10",
  "term_label": "plasma membrane",
  "term_id": "GO:0005886",
  "gene": "UniProtKB:Q9UJ72",
  "gene_name": "Annexin A10"
}